{
  "gene": "UniProtKB:Q7RTX1",
  "gene_symbol": "TAS1R1",
  "term_label": "sensory perception of umami taste",
  "gene_name": "Taste receptor type 1 member 1",
  "term_id": "GO:0050917"
}